{
  "gene_name": "Cyclin-dependent kinase 18",
  "gene_symbol": "CDK18",
  "term_label": "cyclin-dependent protein serine/threonine kinase activity",
  "gene": "UniProtKB:Q07002",
  "term_id": "GO:0004693"
}